{
  "term_label": "phosphatidylinositol binding",
  "term_id": "GO:0035091",
  "gene_symbol": "SNX33",
  "gene_name": "Sorting nexin-33",
  "gene": "UniProtKB:Q8WV41"
}